pallium cell proliferation in forebrain [GO:0022013] (BP) Sources: GOC:cls, GOC:dgh, GOC:dph, GOC:jid, GO_REF:0000021 Definition: The multiplication or reproduction of pallium cells in the forebrain, resulting in the expansion of the cell population. Relationships: is a type of cell proliferation in forebrain [GO:0021846]; is part of GO:0021543